{
  "gene_name": "Tubulin-specific chaperone C",
  "term_label": "protein folding",
  "gene": "UniProtKB:Q15814",
  "term_id": "GO:0006457",
  "gene_symbol": "TBCC"
}